{
  "term_id": "GO:0022625",
  "term_label": "cytosolic large ribosomal subunit",
  "gene_name": "Large ribosomal subunit protein eL31",
  "gene": "UniProtKB:P62899",
  "gene_symbol": "RPL31"
}